{
  "gene_name": "Ribonucleoprotein PTB-binding 2",
  "term_id": "UNKNOWN:0002",
  "term_label": "Unknown biological process",
  "gene": "UniProtKB:Q9HCJ3",
  "gene_symbol": "RAVER2"
}